{
  "gene_name": "Centriolin",
  "term_id": "GO:0005815",
  "gene_symbol": "CNTRL",
  "term_label": "microtubule organizing center",
  "gene": "UniProtKB:Q7Z7A1"
}